{
  "term_label": "proteolysis involved in protein catabolic process",
  "gene": "UniProtKB:O76031",
  "gene_name": "ATP-dependent Clp protease ATP-binding subunit clpX-like, mitochondrial",
  "term_id": "GO:0051603",
  "gene_symbol": "CLPX"
}